neurotransmitter receptor transport [GO:0099637] (biological process) Subtypes: neurotransmitter receptor transport to plasma membrane [GO:0098877], neurotransmitter receptor transport, postsynaptic endosome to lysosome [GO:0098943], neurotransmitter receptor cycle [GO:0099627], GO:0099646, anterograde axonal transport of neurotransmitter receptor complex [GO:0140231] Definition: The directed movement of neurotransmitter receptors. Sources: GOC:dos Relationships: is a type of protein transport [GO:0015031]; is a type of protein-containing complex localization [GO:0031503]